{
  "term_id": "GO:0004222",
  "gene_symbol": "ADAMTS6",
  "gene_name": "A disintegrin and metalloproteinase with thrombospondin motifs 6",
  "gene": "UniProtKB:Q9UKP5",
  "term_label": "metalloendopeptidase activity"
}